histidine decarboxylase activity [GO:0004398] (molecular function) Sources: EC:4.1.1.22 Definition: Catalysis of the reaction: L-histidine = histamine + CO2. Relationships: is a type of carboxy-lyase activity [GO:0016831] Also known as: L-histidine carboxy-lyase (histamine-forming), L-histidine carboxy-lyase activity, L-histidine decarboxylase activity